{
  "gene_name": "Securin",
  "term_label": "nucleus",
  "gene_symbol": "PTTG1",
  "term_id": "GO:0005634",
  "gene": "UniProtKB:O95997"
}